{
  "gene_name": "Coiled-coil domain-containing protein 153",
  "term_id": "UNKNOWN:0001",
  "gene_symbol": "CCDC153",
  "gene": "UniProtKB:Q494R4",
  "term_label": "Unknown molecular function"
}